{
  "gene": "UniProtKB:Q8N609",
  "term_label": "Unknown molecular function",
  "gene_name": "Translocating chain-associated membrane protein 1-like 1",
  "term_id": "UNKNOWN:0001",
  "gene_symbol": "TRAM1L1"
}